dipeptidase activity [GO:0016805] (molecular function) Definition: Catalysis of the hydrolysis of a dipeptide. References: PMID:19879002 Sources: EC:3.4.13.-, https://www.ebi.ac.uk/merops/about/glossary.shtml#DIPEPTIDASE Relationships: is_a exopeptidase activity [GO:0008238] Subtypes: GO:0070573, proline dipeptidase activity [GO:0102009], GO:0160237 Also known as: cytosolic dipeptidase activity